{
  "gene": "UniProtKB:O14493",
  "gene_symbol": "CLDN4",
  "term_label": "paracellular transport",
  "term_id": "GO:0160184",
  "gene_name": "Claudin-4"
}